chloridazon-catechol dioxygenase activity [GO:0047744] (molecular function) Definition: Catalysis of the reaction: 5-amino-4-chloro-2-(2,3-dihydroxyphenyl)pyridazin-3(2H)-one + O2 = 5-amino-4-chloro-2-(2-hydroxymuconoyl)pyridazin-3(2H)-one + 2 H+. Relationships: is a type of oxidoreductase activity, acting on single donors with incorporation of molecular oxygen, incorporation of two atoms of oxygen [GO:0016702] Sources: EC:1.13.11.36, RHEA:20449 Also known as: 5-amino-4-chloro-2-(2,3-dihydroxyphenyl)-3(2H)-pyridazinone 1,2-oxidoreductase (decyclizing)